{
  "gene_name": "WD repeat-containing protein 48",
  "term_label": "double-strand break repair via homologous recombination",
  "gene": "UniProtKB:Q8TAF3",
  "gene_symbol": "WDR48",
  "term_id": "GO:0000724"
}